regulation of translation initiation in response to endoplasmic reticulum stress [GO:0036491] (biological process) Relationships: is a type of regulation of translation in response to endoplasmic reticulum stress [GO:0036490]; is a type of regulation of translational initiation in response to stress [GO:0043558] Subtypes: eiF2alpha phosphorylation in response to endoplasmic reticulum stress [GO:0036492], positive regulation of translation initiation in response to endoplasmic reticulum stress [GO:0036494], GO:0036495, GO:0036497 References: PMID:14676213, PMID:16835242 Sources: GOC:PARL, GOC:bf Also known as: regulation of translation initiation in response to ER stress Definition: Any process that modulates the frequency, rate or extent of translation initiation, as a result of endoplasmic reticulum stress.